activation of meiosis I spindle assembly checkpoint [GO:0090687] (biological process) Definition: Any process that starts the inactive process of a meiosis I cell cycle spindle assembly checkpoint. Sources: GOC:mah Relationships: is a type of positive regulation of meiosis I spindle assembly checkpoint [GO:1905326]